sphingosine-1-phosphate receptor signaling pathway [GO:0003376] (biological process) Relationships: is a type of G protein-coupled receptor signaling pathway [GO:0007186]; is a type of sphingolipid mediated signaling pathway [GO:0090520] Also known as: sphingolipid signaling pathway, sphingolipid signalling pathway, S1P receptor signaling pathway, S1P-activated G-protein coupled receptor signaling pathway, S1P-activated GPCR signaling pathway, S1P-stimulated signal transduction pathway, S1P signaling pathway References: PMID:14592418, PMID:22001186 Sources: GOC:ascb_2009, GOC:signaling Definition: A G protein-coupled receptor signaling pathway initiated by sphingosine-1-phosphate binding to its receptor on the surface of a cell, and ending with the regulation of a downstream cellular process, e.g. transcription.